{
  "gene": "UniProtKB:Q96MC2",
  "term_label": "axonemal dynein complex assembly",
  "gene_name": "Dynein regulatory complex protein 1",
  "gene_symbol": "DRC1",
  "term_id": "GO:0070286"
}